{
  "term_id": "GO:0044233",
  "gene": "UniProtKB:Q969F0",
  "term_label": "mitochondria-associated endoplasmic reticulum membrane contact site",
  "gene_symbol": "FATE1",
  "gene_name": "Fetal and adult testis-expressed transcript protein"
}